{
  "gene": "UniProtKB:Q96DU3",
  "term_id": "UNKNOWN:0001",
  "gene_symbol": "SLAMF6",
  "gene_name": "SLAM family member 6",
  "term_label": "Unknown molecular function"
}